{
  "term_label": "Unknown cellular component",
  "gene_name": "CRACD-like protein",
  "term_id": "UNKNOWN:0003",
  "gene": "UniProtKB:Q6NV74",
  "gene_symbol": "CRACDL"
}